{
  "gene": "UniProtKB:Q99541",
  "gene_symbol": "PLIN2",
  "term_label": "lipid droplet",
  "gene_name": "Perilipin-2",
  "term_id": "GO:0005811"
}